{
  "gene_symbol": "SP2",
  "term_label": "DNA-binding transcription factor activity, RNA polymerase II-specific",
  "gene": "UniProtKB:Q02086",
  "gene_name": "Transcription factor Sp2",
  "term_id": "GO:0000981"
}